sorbitol-6-phosphate 2-dehydrogenase activity [GO:0009010] (molecular function) Definition: Catalysis of the reaction: D-sorbitol 6-phosphate + NAD+ = D-fructose 6-phosphate + NADH + H+. Sources: EC:1.1.1.140 Also known as: D-glucitol-6-phosphate dehydrogenase activity, D-sorbitol 6-phosphate dehydrogenase activity, D-sorbitol-6-phosphate dehydrogenase activity, D-sorbitol-6-phosphate:NAD+ 2-oxidoreductase activity, glucitol-6-phosphate dehydrogenase activity, ketosephosphate reductase activity, sorbitol-6-P-dehydrogenase activity Relationships: is a type of oxidoreductase activity, acting on the CH-OH group of donors, NAD or NADP as acceptor [GO:0016616]